{
  "gene_symbol": "HEATR4",
  "gene_name": "HEAT repeat-containing protein 4",
  "term_label": "oxidoreductase activity",
  "term_id": "GO:0016491",
  "gene": "UniProtKB:Q86WZ0"
}